guanosine-containing compound biosynthetic process [GO:1901070] (biological process) Relationships: is a type of purine ribonucleoside biosynthetic process [GO:0046129] Sources: GOC:TermGenie Definition: The chemical reactions and pathways resulting in the formation of guanosine-containing compounds (guanosines). Also known as: guanosine-containing compound anabolism, guanosine-containing compound biosynthesis, guanosine-containing compound formation, guanosine-containing compound synthesis, guanosines anabolism, guanosines biosynthesis, guanosines biosynthetic process, guanosines formation, guanosines synthesis Subtypes: guanosine biosynthetic process [GO:0046114], 7-methylguanosine biosynthetic process [GO:0046118]